mitochondrial isoleucyl-tRNA aminoacylation [GO:0070152] (BP) Relationships: is a type of GO:0006428; is a type of tRNA aminoacylation for mitochondrial protein translation [GO:0070127] Sources: GOC:mah, GOC:mcc Definition: The process of coupling isoleucine to isoleucyl-tRNA in a mitochondrion, catalyzed by isoleucyl-tRNA synthetase. In tRNA aminoacylation, the amino acid is first activated by linkage to AMP and then transferred to either the 2'- or the 3'-hydroxyl group of the 3'-adenosine residue of the tRNA.